amyloid precursor protein biosynthetic process [GO:0042983] (biological process) Definition: The chemical reactions and pathways resulting in the formation of amyloid precursor protein (APP), the precursor of amyloid-beta, a glycoprotein associated with Alzheimer's disease. Relationships: is a type of macromolecule biosynthetic process [GO:0009059]; is a type of amyloid precursor protein metabolic process [GO:0042982] Sources: GOC:go_curators Regulation: RO_0002211 by regulation of amyloid precursor protein biosynthetic process [GO:0042984]; RO_0002212 by negative regulation of amyloid precursor protein biosynthetic process [GO:0042985]; positively regulated by positive regulation of amyloid precursor protein biosynthetic process [GO:0042986] Also known as: APP biosynthesis, APP biosynthetic process, amyloid precursor protein anabolism, amyloid precursor protein biosynthesis, amyloid precursor protein formation, amyloid precursor protein synthesis